TIS granule [GO:0140363] (cellular component) Definition: A ribonucleoprotein granule located in the cytoplasm that is formed by the RNA-binding protein TIS11B and RNA molecules, enriched in membrane protein-encoding mRNAs with multiple AU-rich elements. TIS granules are reticular meshworks intertwined with the endoplasmic reticulum (ER). Relationships: is a type of GO:0036464 References: PMID:30449617, PMID:30479375 Sources: Wikipedia:TIGER_domain